{
  "gene_name": "Transcription elongation factor A N-terminal and central domain-containing protein",
  "term_label": "nucleus",
  "gene_symbol": "TCEANC",
  "gene": "UniProtKB:Q8N8B7",
  "term_id": "GO:0005634"
}